negative regulation of peptidase activity [GO:0010466] (biological process) Definition: Any process that stops or reduces the rate of peptidase activity, the hydrolysis of peptide bonds within proteins. Sources: GOC:dph, GOC:tb Subtypes: negative regulation of endopeptidase activity [GO:0010951], negative regulation of serine-type peptidase activity [GO:1902572], negative regulation of metallopeptidase activity [GO:1905049] Relationships: is a type of negative regulation of proteolysis [GO:0045861]; is a type of negative regulation of hydrolase activity [GO:0051346]; is a type of regulation of peptidase activity [GO:0052547]; negatively regulates GO:0008233